{
  "gene": "UniProtKB:Q9UJ72",
  "term_label": "nucleus",
  "gene_name": "Annexin A10",
  "term_id": "GO:0005634",
  "gene_symbol": "ANXA10"
}